geraniol biosynthetic process [GO:1903448] (biological process) References: PMID:23200656 Sources: GOC:TermGenie, GOC:di, GO_REF:0000068 Relationships: is a type of polyprenol biosynthetic process [GO:0016094]; is a type of monoterpenoid biosynthetic process [GO:0016099]; is a type of primary alcohol biosynthetic process [GO:0034309]; is a type of olefinic compound biosynthetic process [GO:0120255] Also known as: geraniol anabolism, geraniol biosynthesis, geraniol formation, geraniol synthesis Definition: The chemical reactions and pathways resulting in the formation of geraniol.